{
  "term_id": "GO:0005102",
  "gene_name": "Tyrosine-protein kinase HCK",
  "gene": "UniProtKB:P08631",
  "gene_symbol": "HCK",
  "term_label": "signaling receptor binding"
}